positive regulation of cell communication by electrical coupling [GO:0010650] (biological process) Definition: Any process that increases the frequency, rate or extent of cell communication via electrical coupling. Cell communication via electrical coupling is the process that mediates signaling interactions between one cell and another cell by transfer of current between their adjacent cytoplasms via intercellular protein channels. Sources: GOC:dph, GOC:kmv, GOC:tb Relationships: is a type of positive regulation of cell communication [GO:0010647]; is a type of GO:0010649; positively regulates GO:0010644 Subtypes: positive regulation of cell communication by electrical coupling involved in cardiac conduction [GO:1901846]